{
  "term_label": "Unknown molecular function",
  "gene": "UniProtKB:Q96RU3",
  "gene_symbol": "FNBP1",
  "term_id": "UNKNOWN:0001",
  "gene_name": "Formin-binding protein 1"
}